{
  "gene_symbol": "ANKRD28",
  "term_label": "Unknown cellular component",
  "term_id": "UNKNOWN:0003",
  "gene": "UniProtKB:O15084",
  "gene_name": "Serine_threonine-protein phosphatase 6 regulatory ankyrin repeat subunit A"
}